regulation of timing of anagen [GO:0051884] (biological process) Sources: GOC:ai, GOC:pr Also known as: regulation of anagen Definition: Any process that modulates the frequency, rate or extent of timing of anagen, the growth phase of the hair cycle. Subtypes: positive regulation of timing of anagen [GO:0051885], GO:0051886 Relationships: is a type of GO:0048819; regulates anagen [GO:0042640]